{
  "gene": "UniProtKB:Q9UPR0",
  "term_id": "GO:0007214",
  "gene_name": "Inactive phospholipase C-like protein 2",
  "gene_symbol": "PLCL2",
  "term_label": "gamma-aminobutyric acid signaling pathway"
}